{
  "gene": "UniProtKB:P02747",
  "term_label": "Unknown molecular function",
  "term_id": "UNKNOWN:0001",
  "gene_symbol": "C1QC",
  "gene_name": "Complement C1q subcomponent subunit C"
}